{
  "gene": "UniProtKB:Q0P6D6",
  "gene_name": "Coiled-coil domain-containing protein 15",
  "gene_symbol": "CCDC15",
  "term_label": "Unknown biological process",
  "term_id": "UNKNOWN:0002"
}